{
  "gene_name": "Protein unc-13 homolog B",
  "gene_symbol": "UNC13B",
  "term_id": "GO:0031594",
  "gene": "UniProtKB:O14795",
  "term_label": "neuromuscular junction"
}